{
  "gene_symbol": "TSNARE1",
  "gene": "UniProtKB:Q96NA8",
  "term_id": "GO:0006886",
  "gene_name": "t-SNARE domain-containing protein 1",
  "term_label": "intracellular protein transport"
}